{
  "gene_name": "Cytosolic acyl coenzyme A thioester hydrolase",
  "gene_symbol": "ACOT7",
  "gene": "UniProtKB:O00154",
  "term_label": "long-chain fatty acyl-CoA hydrolase activity",
  "term_id": "GO:0052816"
}